negative regulation of anion channel activity [GO:0010360] (biological process) References: PMID:17319842 Relationships: is a type of GO:0032413; is a type of GO:1903960; negatively regulates monoatomic anion channel activity [GO:0005253] Definition: Any process that stops, prevents, or reduces the frequency, rate, or extent of the anion channel activity.